regulation of Wnt protein secretion [GO:0061356] (biological process) Relationships: is a type of regulation of cell communication [GO:0010646]; is a type of GO:0023051; is a type of regulation of protein secretion [GO:0050708]; regulates GO:0061355 Definition: Any process that modulates the frequency, rate or extent of the controlled release of a Wnt protein from a cell. References: PMID:19223472 Sources: GOC:bf Subtypes: positive regulation of Wnt protein secretion [GO:0061357], negative regulation of Wnt protein secretion [GO:0061358]